inositol-2,4,5-triphosphate 5-phosphatase activity [GO:1990640] (molecular function) Relationships: is a type of inositol trisphosphate phosphatase activity [GO:0046030] Definition: Catalysis of the reaction: 1D-myo-inositol 2,4,5-trisphosphate + H2O = 1D-myo-inositol 2,4-bisphosphate + phosphate. References: PMID:15316017